{
  "term_label": "cytoplasmic dynein complex",
  "gene_symbol": "DYNLRB1",
  "term_id": "GO:0005868",
  "gene": "UniProtKB:Q9NP97",
  "gene_name": "Dynein light chain roadblock-type 1"
}